{
  "gene_symbol": "XAGE2",
  "gene_name": "X antigen family member 2",
  "gene": "UniProtKB:Q96GT9",
  "term_label": "Unknown molecular function",
  "term_id": "UNKNOWN:0001"
}